{
  "gene_symbol": "USP17L8",
  "gene": "UniProtKB:P0C7I0",
  "term_label": "nucleus",
  "gene_name": "Inactive ubiquitin carboxyl-terminal hydrolase 17-like protein 8",
  "term_id": "GO:0005634"
}